{
  "gene_name": "Homeobox protein Nkx-3.2",
  "term_id": "GO:0030154",
  "term_label": "cell differentiation",
  "gene_symbol": "NKX3-2",
  "gene": "UniProtKB:P78367"
}